{
  "gene_name": "von Hippel-Lindau-like protein",
  "gene_symbol": "VHLL",
  "term_id": "UNKNOWN:0002",
  "term_label": "Unknown biological process",
  "gene": "UniProtKB:Q6RSH7"
}